photosystem I reaction center [GO:0009538] (cellular component) Relationships: is a type of membrane protein complex [GO:0098796]; is part of photosystem I [GO:0009522] Sources: GOC:kd, ISBN:0943088399 Also known as: photosystem I reaction centre Definition: A photochemical system containing P700, the chlorophyll a dimer that functions as a primary electron donor. Functioning as a light-dependent plastocyanin-ferredoxin oxidoreductase, it transfers electrons from plastocyanin to ferredoxin.